{
  "gene": "UniProtKB:A2RU54",
  "term_label": "nucleus",
  "term_id": "GO:0005634",
  "gene_name": "Homeobox protein HMX2",
  "gene_symbol": "HMX2"
}